prostaglandin production involved in inflammatory response [GO:0002539] (biological process) Sources: GOC:add, ISBN:0781735149 Relationships: is_a arachidonate metabolite production involved in inflammatory response [GO:0002538] Also known as: prostaglandin production involved in acute inflammatory response Definition: The synthesis or release of any prostaglandin following a stimulus as part of an inflammatory response, resulting in an increase in its intracellular or extracellular levels.